{
  "gene": "UniProtKB:P69891",
  "gene_name": "Hemoglobin subunit gamma-1",
  "gene_symbol": "HBG1",
  "term_label": "hemoglobin alpha binding",
  "term_id": "GO:0031721"
}